{
  "gene_name": "Cell cycle checkpoint protein RAD17",
  "gene_symbol": "RAD17",
  "term_id": "GO:0005634",
  "gene": "UniProtKB:O75943",
  "term_label": "nucleus"
}